{
  "term_id": "GO:0005886",
  "gene_name": "Disintegrin and metalloproteinase domain-containing protein 7",
  "term_label": "plasma membrane",
  "gene_symbol": "ADAM7",
  "gene": "UniProtKB:Q9H2U9"
}